{
  "term_label": "cell migration",
  "gene": "UniProtKB:P55286",
  "term_id": "GO:0016477",
  "gene_symbol": "CDH8",
  "gene_name": "Cadherin-8"
}